{
  "term_label": "Unknown biological process",
  "term_id": "UNKNOWN:0002",
  "gene_symbol": "IAH1",
  "gene_name": "Isoamyl acetate-hydrolyzing esterase 1 homolog",
  "gene": "UniProtKB:Q2TAA2"
}